{
  "gene_symbol": "DHPS",
  "term_id": "GO:0005737",
  "gene": "UniProtKB:P49366",
  "term_label": "cytoplasm",
  "gene_name": "Deoxyhypusine synthase"
}